{
  "gene_name": "Caspase-4",
  "term_id": "GO:0072558",
  "term_label": "NLRP1 inflammasome complex",
  "gene_symbol": "CASP4",
  "gene": "UniProtKB:P49662"
}